negative regulation of endothelial microparticle formation [GO:2000336] (BP) Relationships: is a type of negative regulation of blood microparticle formation [GO:2000333]; is a type of regulation of endothelial microparticle formation [GO:2000335]; negatively regulates GO:0072565 Sources: GOC:BHF, GOC:mah Definition: Any process that stops, prevents or reduces the frequency, rate or extent of endothelial microparticle formation. Also known as: negative regulation of endothelial microparticle generation, negative regulation of endothelial microparticle release